{
  "gene_symbol": "MBOAT4",
  "gene_name": "Ghrelin O-acyltransferase",
  "term_id": "GO:0005789",
  "gene": "UniProtKB:Q96T53",
  "term_label": "endoplasmic reticulum membrane"
}